N-acetyldiaminopimelate deacetylase activity [GO:0050118] (molecular function) Relationships: is a type of hydrolase activity, acting on carbon-nitrogen (but not peptide) bonds, in linear amides [GO:0016811]; is a type of GO:0019213 Definition: Catalysis of the reaction: H2O + N-acetyl-(2S,6S)-2,6-diaminoheptanedioate = (2S,6S)-2,6-diaminoheptanedioate + acetate. Also known as: 6-N-acetyl-LL-2,6-diaminoheptanedioate amidohydrolase activity, N-acetyl-L-diaminopimelic acid deacylase activity, N-acetyl-LL-diaminopimelate deacylase activity, N6-acetyl-LL-2,6-diaminoheptanedioate amidohydrolase activity Sources: RHEA:20405